{
  "gene": "UniProtKB:Q9NTQ9",
  "gene_symbol": "GJB4",
  "gene_name": "Gap junction beta-4 protein",
  "term_id": "GO:0005922",
  "term_label": "connexin complex"
}